{
  "term_id": "GO:0035694",
  "gene": "UniProtKB:Q8TC71",
  "gene_symbol": "SPATA18",
  "gene_name": "Mitochondria-eating protein",
  "term_label": "mitochondrial protein catabolic process"
}